{
  "gene_symbol": "RCSD1",
  "gene": "UniProtKB:Q6JBY9",
  "term_label": "phosphatidylinositol phosphate binding",
  "gene_name": "CapZ-interacting protein",
  "term_id": "GO:1901981"
}